respiratory tube development [GO:0030323] (biological process) Relationships: is a type of tube development [GO:0035295]; is_a animal organ development [GO:0048513] Definition: The process whose specific outcome is the progression of the respiratory tube over time, from its formation to the mature structure. The respiratory tube is assumed to mean any tube in the respiratory tract. Subtypes: bronchus development [GO:0060433], GO:0060435 Sources: GOC:jid